{
  "term_label": "Unknown cellular component",
  "gene_symbol": "OGFR",
  "term_id": "UNKNOWN:0003",
  "gene": "UniProtKB:Q9NZT2",
  "gene_name": "Opioid growth factor receptor"
}